{
  "term_label": "nucleus",
  "gene": "UniProtKB:P05455",
  "gene_symbol": "SSB",
  "gene_name": "Lupus La protein",
  "term_id": "GO:0005634"
}